{
  "term_id": "GO:0005789",
  "term_label": "endoplasmic reticulum membrane",
  "gene_symbol": "SELENOT",
  "gene": "UniProtKB:P62341",
  "gene_name": "Thioredoxin reductase-like selenoprotein T"
}